protein heterodimerization activity [GO:0046982] (molecular function) Sources: GOC:ai Definition: Binding to a nonidentical protein to form a heterodimer. Relationships: is_a protein dimerization activity [GO:0046983]